regulation of antral ovarian follicle growth [GO:2000387] (biological process) Definition: Any process that modulates the frequency, rate or extent of antral ovarian follicle growth. Subtypes: regulation of cumulus cell differentiation [GO:0045592], positive regulation of antral ovarian follicle growth [GO:2000388] Relationships: is_a regulation of developmental growth [GO:0048638]; is a type of regulation of reproductive process [GO:2000241]; regulates GO:0001547 Sources: GOC:obol